{
  "term_label": "Unknown biological process",
  "gene": "UniProtKB:Q9UN19",
  "gene_symbol": "DAPP1",
  "gene_name": "Dual adapter for phosphotyrosine and 3-phosphotyrosine and 3-phosphoinositide",
  "term_id": "UNKNOWN:0002"
}